adenylate cyclase-activating adrenergic receptor signaling pathway [GO:0071880] (biological process) Sources: GOC:BHF, GOC:mah, GOC:signaling Relationships: is a type of adenylate cyclase-activating G protein-coupled receptor signaling pathway [GO:0007189]; is_a adrenergic receptor signaling pathway [GO:0071875] Regulation: negatively regulated by negative regulation of adenylate cyclase-activating adrenergic receptor signaling pathway [GO:0071878] Definition: An adenylate cyclase-activating G protein-coupled receptor signaling pathway initiated by a ligand binding to an adrenergic receptor on the surface of the target cell, and ending with the regulation of a downstream cellular process. Subtypes: adenylate cyclase-activating adrenergic receptor signaling pathway involved in heart process [GO:0086023] Also known as: activation of adenylate cyclase activity by adrenergic receptor signalling pathway, adrenergic receptor, adenylate cyclase activating pathway, adrenergic receptor, adenylyl cyclase activating pathway, activation of adenylate cyclase activity by adrenergic receptor signaling pathway